{
  "term_id": "GO:0003723",
  "gene_symbol": "APOBEC3G",
  "gene_name": "DNA dC-dU-editing enzyme APOBEC-3G",
  "term_label": "RNA binding",
  "gene": "UniProtKB:Q9HC16"
}